{
  "term_id": "GO:0004623",
  "gene": "UniProtKB:Q6P1J6",
  "gene_name": "Phospholipase B1, membrane-associated",
  "term_label": "phospholipase A2 activity",
  "gene_symbol": "PLB1"
}